{
  "term_id": "GO:0043495",
  "gene_symbol": "NHERF2",
  "term_label": "protein-membrane adaptor activity",
  "gene": "UniProtKB:Q15599",
  "gene_name": "Na(+)_H(+) exchange regulatory cofactor NHE-RF2"
}